{
  "gene_symbol": "UPK1A",
  "term_id": "GO:0005886",
  "gene_name": "Uroplakin-1a",
  "term_label": "plasma membrane",
  "gene": "UniProtKB:O00322"
}